morphine catabolic process [GO:0071273] (biological process) Also known as: morphine breakdown, morphine catabolism, morphine degradation References: PMID:22193538 Sources: GOC:ecd, GOC:mah Relationships: is a type of morphine metabolic process [GO:0071272]; is_a isoquinoline alkaloid catabolic process [GO:0071274] Definition: The chemical reactions and pathways resulting in the breakdown of morphine, 17-methyl-7,8-didehydro-4,5alpha-epoxymorphinan-3,6alpha-diol. Morphine is a highly potent opiate analgesic psychoactive drug obtained form the opium poppy, Papaver somniferum.